oogenesis [GO:0048477] (biological process) Definition: The complete process of formation and maturation of an ovum or female gamete from a primordial female germ cell. Examples of this process are found in Mus musculus and Drosophila melanogaster. Relationships: is a type of germ cell development [GO:0007281]; is a type of female gamete generation [GO:0007292] Regulation: regulated by regulation of oogenesis [GO:1905879]; negatively regulated by GO:1905880; positively regulated by GO:1905881 Sources: GOC:kmv, GOC:mtg_sensu, GOC:pr Also known as: ovum development